{
  "gene_symbol": "HCP5",
  "gene_name": "HLA class I histocompatibility antigen protein P5",
  "term_id": "UNKNOWN:0001",
  "gene": "UniProtKB:Q6MZN7",
  "term_label": "Unknown molecular function"
}